{
  "gene_symbol": "GPLD1",
  "term_label": "Unknown biological process",
  "term_id": "UNKNOWN:0002",
  "gene_name": "Phosphatidylinositol-glycan-specific phospholipase D",
  "gene": "UniProtKB:P80108"
}